{
  "gene_symbol": "ACSL5",
  "term_label": "mitochondrion",
  "term_id": "GO:0005739",
  "gene_name": "Long-chain-fatty-acid--CoA ligase 5",
  "gene": "UniProtKB:Q9ULC5"
}